{
  "gene": "UniProtKB:Q9Y2S7",
  "gene_name": "Polymerase delta-interacting protein 2",
  "term_id": "GO:0070987",
  "gene_symbol": "POLDIP2",
  "term_label": "error-free translesion synthesis"
}